pumilio-response element binding [GO:0062104] (molecular function) Relationships: is a type of RNA binding [GO:0003723] References: PMID:30601114 Definition: Binding to a region of RNA containing a Pumilio-response element element. The consensus sequence for the element is UGUAAAUA. Also known as: PRE binding